{
  "gene_symbol": "NAB1",
  "term_id": "GO:0003712",
  "gene_name": "NGFI-A-binding protein 1",
  "term_label": "transcription coregulator activity",
  "gene": "UniProtKB:Q13506"
}